{
  "gene": "UniProtKB:P39687",
  "gene_symbol": "ANP32A",
  "term_label": "nucleus",
  "gene_name": "Acidic leucine-rich nuclear phosphoprotein 32 family member A",
  "term_id": "GO:0005634"
}